{
  "term_label": "positive regulation of apoptotic signaling pathway",
  "term_id": "GO:2001235",
  "gene_symbol": "TPD52L1",
  "gene": "UniProtKB:Q16890",
  "gene_name": "Tumor protein D53"
}